viral scaffold assembly and maintenance [GO:0046807] (BP) Sources: ISBN:0072370319 Relationships: is a type of viral process [GO:0016032]; is part of GO:0019069 Note: See also the cellular component term 'viral scaffold ; GO:0046806'. Definition: The assembly and maintenance of the viral scaffold around which the viral capsid is constructed.